{
  "gene_name": "Leucine-rich repeat, immunoglobulin-like domain and transmembrane domain-containing protein 3",
  "gene": "UniProtKB:Q3SXY7",
  "term_label": "Unknown biological process",
  "gene_symbol": "LRIT3",
  "term_id": "UNKNOWN:0002"
}